{
  "gene_symbol": "HSPA5",
  "term_id": "GO:0036503",
  "gene_name": "Endoplasmic reticulum chaperone BiP",
  "term_label": "ERAD pathway",
  "gene": "UniProtKB:P11021"
}